L-asparagine biosynthetic process from oxaloacetate [GO:0019266] (biological process) Definition: The chemical reactions and pathways resulting in the formation of asparagine from other compounds, including oxaloacetate. Sources: GOC:go_curators Also known as: asparagine anabolism from oxaloacetate, asparagine formation from oxaloacetate, asparagine synthesis from oxaloacetate Relationships: is a type of oxaloacetate metabolic process [GO:0006107]; is a type of amide catabolic process [GO:0043605]; is a type of GO:0043649; is a type of L-asparagine biosynthetic process [GO:0070981]